{
  "gene_name": "Phenylalanine--tRNA ligase beta subunit",
  "gene": "UniProtKB:Q9NSD9",
  "gene_symbol": "FARSB",
  "term_id": "GO:0006432",
  "term_label": "phenylalanyl-tRNA aminoacylation"
}